{
  "gene_symbol": "PRDX4",
  "gene_name": "Peroxiredoxin-4",
  "term_label": "hydrogen peroxide catabolic process",
  "term_id": "GO:0042744",
  "gene": "UniProtKB:Q13162"
}